{
  "gene_symbol": "GPR31",
  "term_id": "GO:0045125",
  "term_label": "bioactive lipid receptor activity",
  "gene_name": "12-(S)-hydroxy-5,8,10,14-eicosatetraenoic acid receptor",
  "gene": "UniProtKB:O00270"
}